noradrenergic neuron differentiation involved in brainstem development [GO:0003361] (BP) Relationships: is_a noradrenergic neuron differentiation [GO:0003357]; is part of brainstem development [GO:0003360] Definition: The process in which a relatively unspecialized cell acquires specialized features of an noradrenergic neuron that is part of the brainstem. Sources: GOC:dph